sophorosyloxydocosanoate biosynthetic process [GO:0019435] (biological process) Also known as: sophorosyloxydocosanoate anabolism, sophorosyloxydocosanoate biosynthesis, sophorosyloxydocosanoate formation, sophorosyloxydocosanoate synthesis Relationships: is a type of glycolipid biosynthetic process [GO:0009247] Definition: The chemical reactions and pathways resulting in the formation of sophorosyloxydocosanoate, 13-sophorosyloxydocosanoate 6',6''-diacetate. Sources: GOC:ai